{
  "gene": "UniProtKB:Q96J92",
  "term_label": "protein kinase activity",
  "term_id": "GO:0004672",
  "gene_name": "Serine_threonine-protein kinase WNK4",
  "gene_symbol": "WNK4"
}